{
  "term_label": "endoplasmic reticulum to Golgi vesicle-mediated transport",
  "gene_name": "Transmembrane emp24 domain-containing protein 9",
  "gene_symbol": "TMED9",
  "term_id": "GO:0006888",
  "gene": "UniProtKB:Q9BVK6"
}